sperm principal piece [GO:0097228] (cellular component) Sources: GOC:cjm, MP:0009836 Definition: The segment of the sperm flagellum where the mitochondrial sheath ends, and the outer dense fibers (ODFs) associated with outer axonemal doublets 3 and 8 are replaced by the 2 longitudinal columns of the fibrous sheath (FS) which run the length of the principal piece and are stabilized by circumferential ribs. The principal piece makes up ~2/3 of the length of the sperm flagellum and is defined by the presence of the FS and of only 7 (rather than 9) ODFs which taper and then terminate near the distal end of the principal piece. Relationships: is a type of cellular anatomical structure [GO:0110165]; BFO_0000050 GO:0036126